{
  "gene_name": "Uncharacterized protein C11orf87",
  "gene": "UniProtKB:Q6NUJ2",
  "term_label": "Unknown cellular component",
  "gene_symbol": "C11orf87",
  "term_id": "UNKNOWN:0003"
}